{
  "term_id": "GO:0016192",
  "gene_name": "ADP-ribosylation factor-like protein 17",
  "term_label": "vesicle-mediated transport",
  "gene": "UniProtKB:Q8IVW1",
  "gene_symbol": "ARL17A"
}